{
  "gene_symbol": "ACTR1A",
  "gene": "UniProtKB:P61163",
  "term_id": "GO:0005200",
  "term_label": "structural constituent of cytoskeleton",
  "gene_name": "Alpha-centractin"
}